negative regulation of N-terminal peptidyl-lysine acetylation [GO:2000760] (biological process) Sources: GOC:obol Definition: Any process that stops, prevents or reduces the frequency, rate or extent of N-terminal peptidyl-lysine acetylation. Relationships: is a type of GO:1903318; is a type of negative regulation of peptidyl-lysine acetylation [GO:2000757]; is a type of regulation of N-terminal peptidyl-lysine acetylation [GO:2000759]; negatively regulates N-terminal peptidyl-lysine acetylation [GO:0018076]